{
  "term_label": "nucleus",
  "gene": "UniProtKB:Q9Y483",
  "term_id": "GO:0005634",
  "gene_symbol": "MTF2",
  "gene_name": "Metal-response element-binding transcription factor 2"
}